{
  "term_label": "negative regulation of VCP-NPL4-UFD1 AAA ATPase complex assembly",
  "gene_name": "Small VCP_p97-interacting protein",
  "gene": "UniProtKB:Q8NHG7",
  "gene_symbol": "SVIP",
  "term_id": "GO:1904240"
}